{
  "gene": "UniProtKB:Q14210",
  "gene_symbol": "LY6D",
  "term_id": "GO:0030098",
  "term_label": "lymphocyte differentiation",
  "gene_name": "Lymphocyte antigen 6D"
}